{
  "gene_symbol": "RBM3",
  "term_label": "regulation of translation",
  "gene": "UniProtKB:P98179",
  "gene_name": "RNA-binding protein 3",
  "term_id": "GO:0006417"
}